defense response to virus [GO:0051607] (biological process) Sources: GOC:ai Relationships: is a type of defense response [GO:0006952]; is_a response to virus [GO:0009615] Also known as: antiviral response, defence response to virus, defense response to viruses Subtypes: RNAi-mediated antiviral immune response [GO:0009616], suppression of viral release by host [GO:0044790], antiviral innate immune response [GO:0140374] Regulation: negatively regulated by negative regulation of defense response to virus [GO:0050687]; RO_0002211 by regulation of defense response to virus [GO:0050688] Definition: Reactions triggered in response to the presence of a virus that act to protect the cell or organism.